nuclear pore linkers [GO:0044612] (cellular component) Relationships: is a type of nuclear protein-containing complex [GO:0140513]; is part of GO:0005643 References: PMID:18046406, PMID:19524430, PMID:20947011, PMID:22419078 Sources: GOC:dgf Also known as: Nic96 complex, Nup82 complex Definition: A substructure of the nuclear pore complex (NPC) that serves to connect members of the central transport channel (composed of FG-nucleoporins) to the core scaffold (composed of the inner and outer NPC rings). In S. cerevisiae, the linkers are Nic96p and Nup82p. In vertebrates, they are Nup93 and Nup88. Components are arranged in 8-fold symmetrical 'spokes' around the central transport channel. Both linkers can be isolated in association with specific FG-nucleoporins, complexes that are sometimes referred to as the Nic96 complex (Nic96p-Nsp1p-Nup49p-Nup57p) and the Nup82 complex (Nup82p-Nup116p-Nup159p-Gle2p).